{
  "term_id": "GO:0016514",
  "gene_symbol": "SMARCE1",
  "gene_name": "SWI_SNF-related matrix-associated actin-dependent regulator of chromatin subfamily E member 1",
  "gene": "UniProtKB:Q969G3",
  "term_label": "SWI/SNF complex"
}